{
  "term_id": "GO:0005521",
  "gene_name": "Transmembrane protein 201",
  "term_label": "lamin binding",
  "gene_symbol": "TMEM201",
  "gene": "UniProtKB:Q5SNT2"
}